{
  "gene_name": "PIK3R3 upstream open reading frame protein",
  "gene": "UniProtKB:A0A087WWA1",
  "gene_symbol": "P3R3URF",
  "term_id": "UNKNOWN:0003",
  "term_label": "Unknown cellular component"
}